{
  "gene": "UniProtKB:P06307",
  "term_id": "GO:0030424",
  "term_label": "axon",
  "gene_symbol": "CCK",
  "gene_name": "Cholecystokinin"
}